{
  "gene": "UniProtKB:Q8N442",
  "term_id": "GO:0005739",
  "term_label": "mitochondrion",
  "gene_symbol": "GUF1",
  "gene_name": "Translation factor GUF1, mitochondrial"
}